oxidoreductase activity, acting on the CH-CH group of donors [GO:0016627] (molecular function) Also known as: oxidoreductase activity, acting on the CH-CH group of donors, other acceptors Subtypes: succinate dehydrogenase activity [GO:0000104], dihydroorotate dehydrogenase activity [GO:0004152], phytoene dehydrogenase activity [GO:0016166], oxidoreductase activity, acting on the CH-CH group of donors, NAD or NADP as acceptor [GO:0016628], oxidoreductase activity, acting on the CH-CH group of donors, cytochrome as acceptor [GO:0016632], GO:0016634, oxidoreductase activity, acting on the CH-CH group of donors, quinone or related compound as acceptor [GO:0016635], oxidoreductase activity, acting on the CH-CH group of donors, iron-sulfur protein as acceptor [GO:0016636], GO:0018129, peptidyl-thiazoline dehydrogenase activity [GO:0018136], carvone reductase activity [GO:0018494], quinoline 2-oxidoreductase activity [GO:0018523], steroid dehydrogenase activity, acting on the CH-CH group of donors [GO:0033765], isoquinoline 1-oxidoreductase activity [GO:0047121], quinaldate 4-oxidoreductase activity [GO:0047122], quinoline-4-carboxylate 2-oxidoreductase activity [GO:0047123], GO:0047542, cyclohexanone dehydrogenase activity [GO:0047797], all-trans-retinol 13,14-reductase activity [GO:0051786], GO:0051989, oxidoreductase activity, acting on the CH-CH group of donors, with a flavin as acceptor [GO:0052890], protoporphyrinogen oxidase activity [GO:0070818] Sources: EC:1.3.-.- Relationships: is a type of oxidoreductase activity [GO:0016491] Definition: Catalysis of an oxidation-reduction (redox) reaction in which a CH-CH group acts as a hydrogen or electron donor and reduces a hydrogen or electron acceptor.